{
  "gene": "UniProtKB:Q13033",
  "term_label": "postsynapse",
  "gene_name": "Striatin-3",
  "gene_symbol": "STRN3",
  "term_id": "GO:0098794"
}